{
  "gene": "UniProtKB:Q5T6R2",
  "term_label": "Unknown molecular function",
  "gene_name": "Putative phosphatidylinositol 3,4,5-trisphosphate 3-phosphatase TPTE2P1",
  "gene_symbol": "TPTE2P1",
  "term_id": "UNKNOWN:0001"
}